{
  "term_id": "UNKNOWN:0001",
  "term_label": "Unknown molecular function",
  "gene_name": "GTP-binding protein 2",
  "gene_symbol": "GTPBP2",
  "gene": "UniProtKB:Q9BX10"
}